regulation of macrophage tolerance induction [GO:0010932] (biological process) Definition: Any process that modulates the frequency, rate, or extent of macrophage tolerance induction. Relationships: is a type of regulation of tolerance induction [GO:0002643]; regulates macrophage tolerance induction [GO:0010931] Subtypes: positive regulation of macrophage tolerance induction [GO:0010933] Sources: GOC:BHF, GOC:dph, GOC:tb